{
  "gene": "UniProtKB:Q92990",
  "gene_symbol": "GLMN",
  "gene_name": "Glomulin",
  "term_id": "GO:0055105",
  "term_label": "ubiquitin-protein transferase inhibitor activity"
}